epithelial fluid transport [GO:0042045] (biological process) References: PMID:11390830 Sources: GOC:jl Definition: The directed movement of fluid across epithelia. Subtypes: liquid clearance, open tracheal system [GO:0035002], transepithelial water transport [GO:0035377] Relationships: is a type of GO:0042044; is a type of transepithelial transport [GO:0070633]